{
  "term_label": "Unknown biological process",
  "term_id": "UNKNOWN:0002",
  "gene_name": "Putative protein FAM66E",
  "gene": "UniProtKB:P0C841",
  "gene_symbol": "FAM66E"
}